melilotate 3-monooxygenase activity [GO:0050091] (molecular function) Sources: EC:1.14.13.4, RHEA:17669 Also known as: melilotate hydroxylase activity, 2-hydroxyphenylpropionate hydroxylase activity, 2-hydroxyphenylpropionic hydroxylase activity, 3-(2-hydroxyphenyl)propanoate,NADH:oxygen oxidoreductase (3-hydroxylating), melilotic hydroxylase activity Definition: Catalysis of the reaction: 3-(2-hydroxyphenyl)propanoate + H+ + NADH + O2 = 3-(2,3-dihydroxyphenyl)propanoate + H2O + NAD+. Relationships: is_a GO:0016709